{
  "gene_name": "Secretory carrier-associated membrane protein 5",
  "term_label": "trans-Golgi network membrane",
  "gene_symbol": "SCAMP5",
  "gene": "UniProtKB:Q8TAC9",
  "term_id": "GO:0032588"
}